{
  "gene_symbol": "GSK3A",
  "gene_name": "Glycogen synthase kinase-3 alpha",
  "term_label": "regulation of microtubule cytoskeleton organization",
  "term_id": "GO:0070507",
  "gene": "UniProtKB:P49840"
}